{
  "term_label": "ubiquitin protein ligase activity",
  "term_id": "GO:0061630",
  "gene": "UniProtKB:Q9NW38",
  "gene_symbol": "FANCL",
  "gene_name": "E3 ubiquitin-protein ligase FANCL"
}